protein metabolic process [GO:0019538] (biological process) Subtypes: ferredoxin metabolic process [GO:0006124], translation [GO:0006412], proteolysis [GO:0006508], Notch receptor processing [GO:0007220], glycoprotein metabolic process [GO:0009100], hemoglobin metabolic process [GO:0020027], GO:0030091, GO:0030163, holo-[acyl-carrier-protein] biosynthetic process [GO:0031108], granulocyte macrophage colony-stimulating factor production [GO:0032604], hepatocyte growth factor production [GO:0032605], GO:0032641, protein modification process [GO:0036211], lipoprotein metabolic process [GO:0042157], amyloid precursor protein metabolic process [GO:0042982], rhodopsin metabolic process [GO:0046154], protein maturation [GO:0051604], GO:0160307, GO:1901142, cytochrome metabolic process [GO:1903604], amyloid fibril formation [GO:1990000] Regulation: regulated by regulation of protein metabolic process [GO:0051246]; RO_0002213 by positive regulation of protein metabolic process [GO:0051247]; negatively regulated by negative regulation of protein metabolic process [GO:0051248] Relationships: is a type of macromolecule metabolic process [GO:0043170]; is a type of primary metabolic process [GO:0044238] Definition: The chemical reactions and pathways involving a protein. Includes protein modification. Also known as: cellular protein metabolic process, cellular protein metabolism, protein metabolic process and modification, protein metabolism, protein metabolism and modification, multicellular organismal protein metabolic process Note: Note that this term is in the subset of terms that should not be used for direct gene product annotation. Instead, select a child term or, if no appropriate child term exists, please request a new term. Direct annotations to this term may be amended during annotation QC. Sources: GOC:ma